response to streptomycin [GO:0046679] (biological process) Sources: GOC:curators Also known as: streptomycin susceptibility/resistance Subtypes: cellular response to streptomycin [GO:0071239] Relationships: is a type of response to antibiotic [GO:0046677]; is_a response to glycoside [GO:1903416] Definition: Any process that results in a change in state or activity of a cell or an organism (in terms of movement, secretion, enzyme production, gene expression, etc.) as a result of a streptomycin stimulus. Streptomycin is a commonly used antibiotic in cell culture media which acts only on prokaryotes and blocks transition from initiation complex to chain elongating ribosome.